{
  "gene_name": "Nucleolar transcription factor 1",
  "term_id": "GO:0006360",
  "gene": "UniProtKB:P17480",
  "gene_symbol": "UBTF",
  "term_label": "transcription by RNA polymerase I"
}